internal peptidyl-lysine acetylation [GO:0018393] (biological process) Sources: GOC:mah Subtypes: peptidyl-lysine N6-acetylation [GO:0018003], alpha-tubulin acetylation [GO:0071929] Definition: The addition of an acetyl group to a non-terminal lysine residue in a protein. Relationships: is a type of internal protein amino acid acetylation [GO:0006475]; is a type of peptidyl-lysine acetylation [GO:0018394]